{
  "gene_name": "Sorting nexin-24",
  "gene": "UniProtKB:Q9Y343",
  "term_id": "UNKNOWN:0002",
  "gene_symbol": "SNX24",
  "term_label": "Unknown biological process"
}